primary lysosome [GO:0005766] (cellular component) Relationships: is a type of GO:0005764 Sources: GOC:jl, ISBN:0815316194 Subtypes: azurophil granule [GO:0042582] Definition: A lysosome before it has fused with a vesicle or vacuole.